protein localization to mating projection tip [GO:1903260] (biological process) Also known as: protein localisation in mating projection tip, protein localisation to mating projection tip, protein localization in mating projection tip, protein localization to conjugation tube tip, protein localization to shmoo tip Relationships: is a type of protein localization to cell tip [GO:1990151] References: PMID:11952834 Sources: GOC:TermGenie, GO_REF:0000087 Definition: A process in which a protein is transported to, or maintained in, a location within a mating projection tip.